urate transmembrane transporter activity [GO:0015143] (molecular function) Sources: GOC:ai Definition: Enables the transfer of urate from one side of a membrane to the other. Urate is the anion of uric acid, 2,6,8-trioxypurine, the end product of purine metabolism in certain mammals and the main excretory product in uricotelic animals. Also known as: uric acid transmembrane transporter activity Relationships: is a type of salt transmembrane transporter activity [GO:1901702]; is part of GO:0015747